{
  "gene": "UniProtKB:O94953",
  "term_id": "GO:0032454",
  "gene_symbol": "KDM4B",
  "gene_name": "Lysine-specific demethylase 4B",
  "term_label": "histone H3K9 demethylase activity"
}